{
  "gene_symbol": "TTI1",
  "term_label": "Unknown biological process",
  "gene_name": "TELO2-interacting protein 1 homolog",
  "term_id": "UNKNOWN:0002",
  "gene": "UniProtKB:O43156"
}